6-pyruvoyltetrahydropterin 2'-reductase activity [GO:0047028] (MF) Definition: Catalysis of the reaction: NADP+ + 6-lactoyl-5,6,7,8-tetrahydropterin = NADPH + H+ + 6-pyruvoyltetrahydropterin. Sources: EC:1.1.1.220, MetaCyc:1.1.1.220-RXN Also known as: 6-lactoyl-5,6,7,8-tetrahydropterin:NADP+ 2'-oxidoreductase activity, 6-pyruvoyl tetrahydropterin (2'-oxo)reductase activity, 6-pyruvoyl-tetrahydropterin 2'-reductase activity, 6-pyruvoyltetrahydropterin reductase activity, 6PPH4(2'-oxo) reductase activity, pyruvoyl-tetrahydropterin reductase activity Relationships: is a type of GO:0016616